{
  "term_id": "GO:0000978",
  "gene_name": "T-box transcription factor TBX19",
  "gene": "UniProtKB:O60806",
  "term_label": "RNA polymerase II cis-regulatory region sequence-specific DNA binding",
  "gene_symbol": "TBX19"
}